{
  "term_label": "RNA polymerase II preinitiation complex assembly",
  "term_id": "GO:0051123",
  "gene_name": "TATA-box-binding protein-associated factor 11-like protein 9",
  "gene_symbol": "TAF11L9",
  "gene": "UniProtKB:A0A1W2PR64"
}